negative regulation of positive chemotaxis [GO:0050928] (biological process) Definition: Any process that stops, prevents, or reduces the frequency, rate or extent of the directed movement of a motile cell or organism towards a higher concentration in a concentration gradient of a specific chemical. Also known as: down regulation of positive chemotaxis, down-regulation of positive chemotaxis, downregulation of positive chemotaxis, inhibition of positive chemotaxis Subtypes: GO:0061123, negative regulation of pollen tube guidance [GO:0160068] Relationships: is a type of negative regulation of chemotaxis [GO:0050922]; is a type of regulation of positive chemotaxis [GO:0050926]; negatively regulates positive chemotaxis [GO:0050918] Sources: GOC:ai